{
  "gene": "UniProtKB:Q2Y0W8",
  "gene_symbol": "SLC4A8",
  "term_id": "GO:0051453",
  "term_label": "regulation of intracellular pH",
  "gene_name": "Electroneutral sodium bicarbonate exchanger 1"
}